{
  "gene": "UniProtKB:Q9BRD0",
  "term_id": "UNKNOWN:0001",
  "gene_name": "BUD13 homolog",
  "term_label": "Unknown molecular function",
  "gene_symbol": "BUD13"
}